neurotrophin binding [GO:0043121] (molecular function) Definition: Binding to a neurotrophin, any of a family of growth factors that prevent apoptosis in neurons and promote nerve growth. Sources: GOC:jl Also known as: neurotrophic factor binding, NT 4/5 binding, NT-3 binding, NT-4 binding, NT-4/5 binding, NT-5 binding, NT3 binding, NT4 binding, NT5 binding, neurotrophin 3 binding, neurotrophin 4/5 binding, neurotrophin-3 binding, neurotrophin-4/5 binding, neurotrophin TRK receptor activity, neurotrophin TRKA receptor activity, neurotrophin TRKB receptor activity, neurotrophin TRKC receptor activity Note: Note that mammalian NT-5 was initially named differently from amphibian NT-4 because of sequence differences, but the two genes were later shown to be functionally equivalent [SF:919858]. Relationships: is a type of growth factor binding [GO:0019838] Subtypes: brain-derived neurotrophic factor binding [GO:0048403], nerve growth factor binding [GO:0048406]